{
  "gene_name": "Carbohydrate sulfotransferase 7",
  "gene_symbol": "CHST7",
  "gene": "UniProtKB:Q9NS84",
  "term_label": "chondroitin sulfate proteoglycan biosynthetic process",
  "term_id": "GO:0050650"
}